{
  "gene": "UniProtKB:A6NEV1",
  "gene_name": "Proline-rich protein 23A",
  "term_label": "Unknown molecular function",
  "gene_symbol": "PRR23A",
  "term_id": "UNKNOWN:0001"
}